{
  "gene_name": "Ankyrin repeat domain-containing protein 34B",
  "term_id": "UNKNOWN:0002",
  "term_label": "Unknown biological process",
  "gene_symbol": "ANKRD34B",
  "gene": "UniProtKB:A5PLL1"
}